negatively regulates [RO:0002212] (external) Relationships: subPropertyOf regulates [RO:0002211]